{
  "gene_name": "Putative pancreatic polypeptide 2",
  "gene": "UniProtKB:Q9NRI7",
  "term_id": "UNKNOWN:0003",
  "gene_symbol": "PPY2P",
  "term_label": "Unknown cellular component"
}